egg activation [GO:0007343] (biological process) Definition: The process in which the egg becomes metabolically active, initiates protein and DNA synthesis and undergoes structural changes to its cortex and/or cytoplasm. References: PMID:9630751 Sources: GOC:bf Relationships: is a type of cell activation [GO:0001775]; is part of single fertilization [GO:0007338]